{
  "term_label": "GTPase activator activity",
  "gene_name": "SLIT-ROBO Rho GTPase-activating protein 2C",
  "gene": "UniProtKB:P0DJJ0",
  "gene_symbol": "SRGAP2C",
  "term_id": "GO:0005096"
}